dopamine receptor binding [GO:0050780] (molecular function) Relationships: is a type of G protein-coupled receptor binding [GO:0001664] Sources: GOC:ai Definition: Binding to a dopamine receptor. Subtypes: GO:0031748, D2 dopamine receptor binding [GO:0031749], D3 dopamine receptor binding [GO:0031750], GO:0031751, D5 dopamine receptor binding [GO:0031752]